{
  "term_id": "GO:0003730",
  "gene": "UniProtKB:A0A2R8Y4L2",
  "gene_name": "Heterogeneous nuclear ribonucleoprotein A1-like 3",
  "term_label": "mRNA 3'-UTR binding",
  "gene_symbol": "HNRNPA1L3"
}